{
  "term_label": "calcium ion binding",
  "gene_name": "Allograft inflammatory factor 1",
  "term_id": "GO:0005509",
  "gene": "UniProtKB:P55008",
  "gene_symbol": "AIF1"
}